amine transmembrane transporter activity [GO:0005275] (molecular function) Sources: GOC:mtg_transport, ISBN:0198506732, ISBN:0815340729 Subtypes: methylammonium transmembrane transporter activity [GO:0015200], GO:0034228 Also known as: amine/amide/polyamine channel activity, amine/polyamine transmembrane transporter activity, amino acid-polyamine transmembrane transporter activity Definition: Enables the transfer of amines, including polyamines, from one side of a membrane to the other. Amines are organic compounds that are weakly basic in character and contain an amino (-NH2) or substituted amino group. Relationships: is a type of GO:0022857; is part of amine transport [GO:0015837]